{
  "term_label": "Unknown molecular function",
  "gene": "UniProtKB:P53990",
  "gene_name": "IST1 homolog",
  "term_id": "UNKNOWN:0001",
  "gene_symbol": "IST1"
}